L-arabinose metabolic process [GO:0046373] (biological process) Also known as: L-arabinose metabolism Subtypes: L-arabinose catabolic process [GO:0019572], L-arabinose biosynthetic process [GO:0033357] Sources: GOC:jsg, GOC:mah, ISBN:0198506732 Definition: The chemical reactions and pathways involving L-arabinose, the D-enantiomer of arabino-pentose. L-arabinose occurs free, e.g. in the heartwood of many conifers, and in the combined state, in both furanose and pyranose forms, as a constituent of various plant hemicelluloses, bacterial polysaccharides etc. Relationships: is a type of arabinose metabolic process [GO:0019566]